translation initiation factor binding [GO:0031369] (molecular function) Sources: GOC:mah Subtypes: eukaryotic initiation factor 4E binding [GO:0008190], eukaryotic initiation factor 4G binding [GO:0031370], GO:0071074 Definition: Binding to a translation initiation factor, any polypeptide factor involved in the initiation of ribosome-mediated translation. Relationships: is a type of protein binding [GO:0005515]